{
  "gene_symbol": "GRB2",
  "gene": "UniProtKB:P62993",
  "term_label": "regulation of MAPK cascade",
  "gene_name": "Growth factor receptor-bound protein 2",
  "term_id": "GO:0043408"
}